cellular response to prostaglandin E stimulus [GO:0071380] (biological process) Sources: GOC:mah Relationships: is_a GO:0034695; is a type of cellular response to prostaglandin stimulus [GO:0071379]; is a type of cellular response to alcohol [GO:0097306]; is a type of cellular response to ketone [GO:1901655] Definition: Any process that results in a change in state or activity of a cell (in terms of movement, secretion, enzyme production, gene expression, etc.) as a result of a prostagladin E stimulus.